2-coumarate reductase activity [GO:0047788] (molecular function) Definition: Catalysis of the reaction: 3-(2-hydroxyphenyl)propanoate + NAD+ = trans-2-coumarate + H+ + NADH. Also known as: coumarate reductase activity, 3-(2-hydroxyphenyl)propanoate:NAD+ oxidoreductase activity, melilotate dehydrogenase activity Relationships: is a type of GO:0016628 Sources: EC:1.3.1.11, RHEA:21444